cellular response to inositol starvation [GO:0036110] (biological process) References: PMID:19606215 Sources: GOC:al Relationships: is a type of cellular response to starvation [GO:0009267] Definition: Any process that results in a change in state or activity of a cell (in terms of movement, secretion, enzyme production, gene expression, etc.) as a result of deprivation of inositol.